{
  "term_id": "GO:0003682",
  "gene_name": "Testis-specific Y-encoded-like protein 2",
  "gene_symbol": "TSPYL2",
  "gene": "UniProtKB:Q9H2G4",
  "term_label": "chromatin binding"
}